{
  "gene_symbol": "SYT10",
  "term_id": "GO:0007268",
  "term_label": "chemical synaptic transmission",
  "gene": "UniProtKB:Q6XYQ8",
  "gene_name": "Synaptotagmin-10"
}